21S rRNA pseudouridine(2819) synthase activity [GO:0160143] (MF) Sources: EC:5.4.99.43, RHEA:42556 Relationships: is a type of GO:0120159 Definition: Catalysis of the reaction: uridine(2819) in 21S rRNA = pseudouridine(2819) in 21S rRNA.